{
  "gene_name": "Semaphorin-3B",
  "gene": "UniProtKB:Q13214",
  "gene_symbol": "SEMA3B",
  "term_label": "neuropilin binding",
  "term_id": "GO:0038191"
}